{
  "term_label": "microtubule cytoskeleton organization",
  "gene_symbol": "EML2",
  "gene": "UniProtKB:O95834",
  "gene_name": "Echinoderm microtubule-associated protein-like 2",
  "term_id": "GO:0000226"
}